{
  "gene_symbol": "COPA",
  "term_label": "endoplasmic reticulum to Golgi vesicle-mediated transport",
  "term_id": "GO:0006888",
  "gene_name": "Coatomer subunit alpha",
  "gene": "UniProtKB:P53621"
}